{
  "gene_name": "Rho-related GTP-binding protein RhoB",
  "term_label": "plasma membrane",
  "term_id": "GO:0005886",
  "gene_symbol": "RHOB",
  "gene": "UniProtKB:P62745"
}